MAPK-activating adrenergic receptor signaling pathway [GO:0071883] (biological process) Relationships: is a type of adrenergic receptor signaling pathway [GO:0071875] Also known as: activation of MAP kinase activity by adrenergic receptor signaling pathway, activation of MAP kinase activity by adrenergic receptor signalling pathway, activation of MAPK activity by adrenergic receptor signaling pathway, activation of MAPK activity by adrenergic receptor signalling pathway Definition: The series of molecular signals generated as a consequence of an adrenergic receptor binding to its physiological ligand and leading to the activation of a MAP kinase cascade. Sources: GOC:BHF, GOC:mah